{
  "term_label": "kinase binding",
  "gene_name": "Leucine-rich repeat-containing protein 14",
  "gene_symbol": "LRRC14",
  "term_id": "GO:0019900",
  "gene": "UniProtKB:Q15048"
}